{
  "gene_name": "Zinc finger SWIM domain-containing protein 4",
  "term_label": "Unknown biological process",
  "term_id": "UNKNOWN:0002",
  "gene_symbol": "ZSWIM4",
  "gene": "UniProtKB:Q9H7M6"
}